{
  "term_label": "nucleus",
  "term_id": "GO:0005634",
  "gene_name": "Histone-lysine N-methyltransferase SUV39H2",
  "gene": "UniProtKB:Q9H5I1",
  "gene_symbol": "SUV39H2"
}